{
  "gene_symbol": "CASP7",
  "gene_name": "Caspase-7",
  "gene": "UniProtKB:P55210",
  "term_label": "execution phase of apoptosis",
  "term_id": "GO:0097194"
}